{
  "gene": "UniProtKB:Q5T7M9",
  "gene_name": "Divergent protein kinase domain 1A",
  "term_label": "Unknown biological process",
  "term_id": "UNKNOWN:0002",
  "gene_symbol": "DIPK1A"
}